regulation of growth [GO:0040008] (biological process) Relationships: is a type of regulation of biological process [GO:0050789]; regulates GO:0040007 Definition: Any process that modulates the frequency, rate or extent of the growth of all or part of an organism so that it occurs at its proper speed, either globally or in a specific part of the organism's development. Sources: GOC:ems, GOC:mah Subtypes: regulation of cell growth [GO:0001558], regulation of budding cell apical bud growth [GO:0010568], regulation of filamentous growth [GO:0010570], GO:0035212, regulation of growth rate [GO:0040009], negative regulation of growth [GO:0045926], positive regulation of growth [GO:0045927], regulation of developmental growth [GO:0048638], regulation of secondary growth [GO:2000603]